phosphatidylinositol phosphate binding [GO:1901981] (MF) Relationships: is a type of phosphatidylinositol binding [GO:0035091] Definition: Binding to phosphatidylinositol phosphate. References: PMID:23445487 Sources: GOC:TermGenie Subtypes: phosphatidylinositol-3,4,5-trisphosphate binding [GO:0005547], GO:0010314, phosphatidylinositol-3-phosphate binding [GO:0032266], phosphatidylinositol-4-phosphate binding [GO:0070273], phosphatidylinositol bisphosphate binding [GO:1902936]